adaptive immune memory response [GO:0090716] (biological process) References: PMID:26831526 Sources: GOC:add Subtypes: GO:0090717 Definition: An immune response directed against a previously encountered antigen, being quicker and quantitatively better compared with the primary response. Relationships: is a type of GO:0002250; is a type of immunological memory process [GO:0090713] Regulation: regulated by GO:1905674; negatively regulated by negative regulation of adaptive immune memory response [GO:1905675]; positively regulated by positive regulation of adaptive immune memory response [GO:1905676]